{
  "gene_name": "Syntaxin-16",
  "gene": "UniProtKB:O14662",
  "term_id": "GO:0006886",
  "gene_symbol": "STX16",
  "term_label": "intracellular protein transport"
}